positive regulation of macrophage tolerance induction [GO:0010933] (BP) Definition: Any process that increases the frequency, rate, or extent of B cell tolerance induction. Sources: GOC:BHF, GOC:dph, GOC:tb Relationships: is a type of positive regulation of tolerance induction [GO:0002645]; is a type of regulation of macrophage tolerance induction [GO:0010932]; RO_0002213 GO:0010931